{
  "gene_symbol": "GOLPH3L",
  "gene": "UniProtKB:Q9H4A5",
  "term_label": "phosphatidylinositol-4-phosphate binding",
  "gene_name": "Golgi phosphoprotein 3-like",
  "term_id": "GO:0070273"
}